response to vitamin E [GO:0033197] (biological process) Sources: GOC:sl Relationships: is a type of GO:0033273; is a type of GO:1901700 Also known as: response to DL-alpha-tocopherol acetate, response to DL-alpha-tocopheryl acetate, response to O-Acetyl-alpha-tocopherol Definition: Any process that results in a change in state or activity of a cell or an organism (in terms of movement, secretion, enzyme production, gene expression, etc.) as a result of a vitamin E stimulus. Subtypes: cellular response to vitamin E [GO:0071306]